negative regulation of T-helper 17 cell lineage commitment [GO:2000329] (biological process) Also known as: negative regulation of T-helper 17 cell fate commitment, negative regulation of Th17 cell lineage commitment, negative regulation of Th17 fate commitment Sources: GOC:BHF, GOC:mah Definition: Any process that stops, prevents or reduces the frequency, rate or extent of T-helper 17 cell lineage commitment. Relationships: is_a negative regulation of cell fate commitment [GO:0010454]; is a type of negative regulation of T-helper 17 cell differentiation [GO:2000320]; is a type of regulation of T-helper 17 cell lineage commitment [GO:2000328]; negatively regulates GO:0072540